{
  "gene_symbol": "FAM181A",
  "term_id": "UNKNOWN:0002",
  "term_label": "Unknown biological process",
  "gene": "UniProtKB:Q8N9Y4",
  "gene_name": "Protein FAM181A"
}